{
  "term_id": "GO:0007015",
  "gene_symbol": "KASH5",
  "term_label": "actin filament organization",
  "gene_name": "Protein KASH5",
  "gene": "UniProtKB:Q8N6L0"
}